{
  "term_label": "receptor complex",
  "gene_name": "Epidermal growth factor receptor",
  "gene": "UniProtKB:P00533",
  "gene_symbol": "EGFR",
  "term_id": "GO:0043235"
}